{
  "term_label": "negative regulation of Wnt signaling pathway",
  "gene": "UniProtKB:Q9NSA3",
  "term_id": "GO:0030178",
  "gene_name": "Beta-catenin-interacting protein 1",
  "gene_symbol": "CTNNBIP1"
}